{
  "gene_symbol": "KRT78",
  "term_id": "GO:0030280",
  "gene": "UniProtKB:Q8N1N4",
  "gene_name": "Keratin, type II cytoskeletal 78",
  "term_label": "structural constituent of skin epidermis"
}